{
  "gene": "UniProtKB:P00480",
  "term_label": "citrulline biosynthetic process",
  "term_id": "GO:0019240",
  "gene_name": "Ornithine transcarbamylase, mitochondrial",
  "gene_symbol": "OTC"
}